organelle subcompartment [GO:0031984] (cellular component) Relationships: is a type of cellular anatomical structure [GO:0110165]; is part of membrane-bounded organelle [GO:0043227]; is part of intracellular organelle [GO:0043229] Note: Note that this term refers to membrane-bounded compartments that are not considered organelles in their own right, but form parts of larger organelles. Definition: A compartment that consists of a lumen and an enclosing membrane, and is part of an organelle. Also known as: suborganelle compartment Sources: GOC:mah, GOC:pz Subtypes: GO:0032046, Golgi apparatus subcompartment [GO:0098791], endoplasmic reticulum subcompartment [GO:0098827]